{
  "term_id": "UNKNOWN:0001",
  "gene_symbol": "GPR82",
  "gene_name": "Probable G-protein coupled receptor 82",
  "gene": "UniProtKB:Q96P67",
  "term_label": "Unknown molecular function"
}